Golgi-associated vesicle [GO:0005798] (cellular component) Relationships: is_a cytoplasmic vesicle [GO:0031410] Definition: Any vesicle associated with the Golgi complex and involved in mediating transport within the Golgi or between the Golgi and other parts of the cell. Also known as: Golgi vesicle, vesicular component Subtypes: COPI-coated vesicle [GO:0030137], trans-Golgi network transport vesicle [GO:0030140] Note: Note that this definition includes vesicles that are transiently associated with the Golgi. Sources: GOC:mah